S100A8 complex [GO:1990661] (cellular component) Definition: A protein complex composed of a S100A8 dimer and capable of binding to toll-like receptor 4 (TLR4). References: PMID:25417112 Sources: GOC:bhm Also known as: S100A8 homodimer Note: An example of this is S100A8 in human (UniProt symbol P27005) in PMID:25417112 (inferred from direct assay). Relationships: is a type of protein-containing complex [GO:0032991]